{
  "term_id": "GO:0043123",
  "term_label": "positive regulation of canonical NF-kappaB signal transduction",
  "gene_symbol": "CD40LG",
  "gene_name": "CD40 ligand",
  "gene": "UniProtKB:P29965"
}